positive regulation of protein targeting to mitochondrion [GO:1903955] (biological process) Relationships: is a type of GO:1903214; is a type of positive regulation of establishment of protein localization to mitochondrion [GO:1903749]; positively regulates protein targeting to mitochondrion [GO:0006626] Note: An example of this is PINK1 in human (UniProt symbol Q9BXM7) in PMID:24270810 inferred from mutant phenotype. Definition: Any process that activates or increases the frequency, rate or extent of protein targeting to mitochondrion. References: PMID:24270810 Sources: GOC:PARL, GOC:TermGenie, GOC:pad, GO_REF:0000058 Subtypes: positive regulation of protein insertion into mitochondrial outer membrane [GO:1903638] Also known as: positive regulation of protein import into mitochondrion, positive regulation of protein targeting to mitochondria, positive regulation of protein-mitochondrial targeting, up regulation of protein import into mitochondrion, up regulation of protein targeting to mitochondria, up regulation of protein targeting to mitochondrion, up regulation of protein-mitochondrial targeting, up-regulation of protein import into mitochondrion, up-regulation of protein targeting to mitochondria, up-regulation of protein targeting to mitochondrion, up-regulation of protein-mitochondrial targeting, upregulation of protein import into mitochondrion, upregulation of protein targeting to mitochondria, upregulation of protein targeting to mitochondrion, upregulation of protein-mitochondrial targeting, activation of protein import into mitochondrion, activation of protein targeting to mitochondria, activation of protein targeting to mitochondrion, activation of protein-mitochondrial targeting, activation of mitochondrial protein import, activation of mitochondrial translocation, positive regulation of mitochondrial protein import, positive regulation of mitochondrial translocation, up regulation of mitochondrial protein import, up regulation of mitochondrial translocation, up-regulation of mitochondrial protein import, up-regulation of mitochondrial translocation, upregulation of mitochondrial protein import, upregulation of mitochondrial translocation